glycoside metabolic process [GO:0016137] (biological process) Sources: ISBN:0198547684 Relationships: is a type of carbohydrate derivative metabolic process [GO:1901135] Subtypes: mycothiol metabolic process [GO:0010126], saponin metabolic process [GO:0016134], GO:0016138, glycoside catabolic process [GO:0016139], coniferin metabolic process [GO:0033491], daunorubicin metabolic process [GO:0044597], doxorubicin metabolic process [GO:0044598], glucosylglycerol metabolic process [GO:0051472], mannosylglycerate metabolic process [GO:0051478], GO:1901038, gentamycin metabolic process [GO:1901128] Also known as: O-glycoside metabolic process, O-glycoside metabolism, glycoside metabolism Definition: The chemical reactions and pathways involving glycosides, compounds in which a glycosyl group is substituted into a hydroxyl, thiol or selenol group in another compound.